negative regulation of microglia differentiation [GO:0014007] (biological process) Sources: GOC:ef Also known as: down regulation of microglia differentiation, down-regulation of microglia differentiation, downregulation of microglia differentiation, negative regulation of microglial cell differentiation, inhibition of microglia differentiation Definition: Any process that stops, prevents, or reduces the frequency, rate or extent of microglia differentiation, the process in which a relatively unspecialized cell acquires specialized features of a microglial cell. Relationships: is a type of GO:0014006; is a type of negative regulation of macrophage differentiation [GO:0045650]; is a type of negative regulation of glial cell differentiation [GO:0045686]; negatively regulates microglia differentiation [GO:0014004]